malate-CoA ligase activity [GO:0050074] (molecular function) Relationships: is a type of GO:0016878 Also known as: malate thiokinase activity, malate:CoA ligase (ADP-forming), malyl coenzyme A synthetase activity, malyl-CoA synthetase activity Sources: EC:6.2.1.9, MetaCyc:MALATE--COA-LIGASE-RXN Definition: Catalysis of the reaction: ATP + malate + CoA = ADP + phosphate + malyl-CoA.